{
  "term_id": "GO:0005886",
  "term_label": "plasma membrane",
  "gene_symbol": "NPY6R",
  "gene": "UniProtKB:Q99463",
  "gene_name": "Putative neuropeptide Y receptor type 6"
}